{
  "gene_symbol": "SCEL",
  "gene_name": "Sciellin",
  "term_id": "GO:0005737",
  "gene": "UniProtKB:O95171",
  "term_label": "cytoplasm"
}